apical ectodermal ridge formation [GO:1905139] (biological process) References: PMID:18359901, PMID:9323126, PMID:9596583 Sources: GOC:TermGenie, GO_REF:0000081 Also known as: apical epidermal ridge formation, AER formation, crista ectodermalis apicalis formation Relationships: is a type of anatomical structure formation involved in morphogenesis [GO:0048646]; is part of appendage morphogenesis [GO:0035107] Definition: The process that gives rise to the apical ectodermal ridge. This process pertains to the initial formation of a structure from unspecified parts. Regulation: regulated by regulation of apical ectodermal ridge formation [GO:1905140]; negatively regulated by GO:1905141; positively regulated by positive regulation of apical ectodermal ridge formation [GO:1905142]